{
  "gene": "UniProtKB:P20336",
  "gene_name": "Ras-related protein Rab-3A",
  "term_id": "GO:0005768",
  "term_label": "endosome",
  "gene_symbol": "RAB3A"
}